{
  "gene": "UniProtKB:Q9GZU2",
  "term_label": "regulation of transcription by RNA polymerase II",
  "gene_symbol": "PEG3",
  "term_id": "GO:0006357",
  "gene_name": "Paternally-expressed gene 3 protein"
}